{
  "gene_symbol": "KRTAP20-3",
  "term_id": "UNKNOWN:0001",
  "term_label": "Unknown molecular function",
  "gene_name": "Keratin-associated protein 20-3",
  "gene": "UniProtKB:Q3LI60"
}